ATP-dependent NAD(P)H-hydrate dehydratase activity [GO:0047453] (molecular function) Relationships: is a type of GO:0016836 Also known as: reduced nicotinamide adenine dinucleotide hydrate dehydratase activity, ATP-dependent H(4)NAD(P)OH dehydratase activity, ATP-dependent H4NAD(P)OH dehydratase activity, (6S)-beta-6-hydroxy-1,4,5,6-tetrahydronicotinamide-adenine-dinucleotide hydro-lyase (ATP-hydrolysing), (6S)-beta-6-hydroxy-1,4,5,6-tetrahydronicotinamide-adenine-dinucleotide hydro-lyase(ATP-hydrolysing; NADH-forming) References: PMID:3061454 Sources: EC:4.2.1.93 Definition: Catalysis of the reaction: (6S)-6beta-hydroxy-1,4,5,6-tetrahydronicotinamide adenine dinucleotide + ATP = ADP + H+ + NAD(P)H + phosphate.